{
  "gene": "UniProtKB:Q6WRX3",
  "term_label": "Unknown molecular function",
  "gene_symbol": "ZYG11A",
  "term_id": "UNKNOWN:0001",
  "gene_name": "Protein zyg-11 homolog A"
}